{
  "gene_name": "Zinc finger protein 771",
  "gene_symbol": "ZNF771",
  "term_label": "regulation of transcription by RNA polymerase II",
  "term_id": "GO:0006357",
  "gene": "UniProtKB:Q7L3S4"
}